anhydrosialidase activity [GO:0033995] (molecular function) Relationships: is a type of carbon-oxygen lyase activity, acting on polysaccharides [GO:0016837] Also known as: anhydroneuraminidase activity, glycoconjugate sialyl-lyase (2,7-cyclizing) activity, sialglycoconjugate N-acylneuraminylhydrolase (2,7-cyclizing) activity, sialidase L activity Sources: EC:4.2.2.15 Definition: Catalysis of the reaction: an N-acetylneuraminate glycoside = 2,7-anhydro-alpha-N-acetylneuraminate + an alpha-sialyl group. This reaction is the elimination of alpha-sialyl groups in N-acetylneuraminic acid glycosides, releasing 2,7-anhydro-alpha-N-acetylneuraminate.